{
  "gene": "UniProtKB:P51681",
  "term_label": "cytoplasm",
  "term_id": "GO:0005737",
  "gene_symbol": "CCR5",
  "gene_name": "C-C chemokine receptor type 5"
}